virus tail, tube [GO:0098026] (CC) References: PMID:33188213 Sources: VZ:3960 Relationships: is_a virion component [GO:0044423]; is part of virus tail [GO:0098015] Note: Applies in particular the Myoviridae bacteriophages. Many bacteriophages with dsDNA genomes, or Caudovirales, have a tail. The viral tail can be short (Podoviridae), long and non-contractile (Siphoviridae) or long and contractile (Myoviridae). The tail is the channel through which the phage genome is injected into the host bacterial cell. Also known as: bacteriophage tail tube Definition: The internal tube of the tail of some viruses. The virus tail tube is the channel for DNA ejection into the host cytoplasm.